{
  "gene": "UniProtKB:A0A804HIB5",
  "gene_symbol": "A0A804HIB5",
  "term_id": "UNKNOWN:0003",
  "term_label": "Unknown cellular component",
  "gene_name": "Uncharacterized protein"
}